{
  "gene_symbol": "RBM24",
  "term_id": "GO:0000381",
  "term_label": "regulation of alternative mRNA splicing, via spliceosome",
  "gene": "UniProtKB:Q9BX46",
  "gene_name": "RNA-binding protein 24"
}